symbiont-mediated suppression of host MAPK cascade [GO:0141070] (biological process) References: PMID:18005697 Relationships: is a type of symbiont-mediated suppression of host signal transduction pathway [GO:0052029]; is a type of symbiont-mediated perturbation of host MAPK cascade [GO:0052080] Also known as: disruption of host MAP kinase signaling pathway, disruption of host MAPK signal transduction pathway, disruption of host MAPK signaling pathway, symbiont-mediated suppression of host MAPK signal transduction pathway Definition: A process in which a symbiont interferes with, inhibits or disrupts a MAPK signal transduction pathway in its host organism. The host is defined as the larger of the organisms involved in a symbiotic interaction.